{
  "gene_symbol": "NUDT15",
  "gene": "UniProtKB:Q9NV35",
  "term_id": "GO:0035539",
  "term_label": "8-oxo-7,8-dihydrodeoxyguanosine triphosphate pyrophosphatase activity",
  "gene_name": "Nucleotide triphosphate diphosphatase NUDT15"
}